{
  "term_label": "Unknown molecular function",
  "gene": "UniProtKB:Q9C0I3",
  "gene_symbol": "CCSER1",
  "gene_name": "Serine-rich coiled-coil domain-containing protein 1",
  "term_id": "UNKNOWN:0001"
}